{
  "term_id": "UNKNOWN:0003",
  "gene_name": "SLIT-ROBO Rho GTPase-activating protein 3",
  "term_label": "Unknown cellular component",
  "gene_symbol": "SRGAP3",
  "gene": "UniProtKB:O43295"
}